{
  "gene_name": "Golgi phosphoprotein 3",
  "gene": "UniProtKB:Q9H4A6",
  "term_label": "trans-Golgi network",
  "term_id": "GO:0005802",
  "gene_symbol": "GOLPH3"
}